EH domain binding [GO:1990175] (molecular function) References: PMID:11911876, PMID:21115825 Sources: GOC:hjd Definition: Binding to an EH domain of a protein. The EH stand for Eps15 homology. This was originally identified as a motif present in three copies at the NH2-termini of Eps15 and of the related molecule Eps15R. Relationships: is_a protein domain specific binding [GO:0019904]